{
  "term_id": "GO:0051082",
  "term_label": "unfolded protein binding",
  "gene_name": "NudC domain-containing protein 2",
  "gene_symbol": "NUDCD2",
  "gene": "UniProtKB:Q8WVJ2"
}